negative regulation of exit from meiosis [GO:0106061] (biological process) Definition: Any process that stops, prevents or reduces the frequency, rate or extent of exit from meiosis. Relationships: is a type of regulation of exit from meiosis [GO:0106060]; is a type of negative regulation of meiotic cell cycle phase transition [GO:1901994]; negatively regulates exit from meiosis [GO:1990947] References: PMID:11493649 Sources: GOC:al